{
  "gene_name": "Mitoregulin",
  "gene": "UniProtKB:Q8NCU8",
  "term_id": "GO:0005743",
  "gene_symbol": "MTLN",
  "term_label": "mitochondrial inner membrane"
}